{
  "gene_name": "cAMP-regulated phosphoprotein 21",
  "term_label": "Unknown molecular function",
  "gene_symbol": "ARPP21",
  "term_id": "UNKNOWN:0001",
  "gene": "UniProtKB:Q9UBL0"
}